{
  "gene_name": "Neurotrophin receptor-interacting factor homolog",
  "gene": "UniProtKB:Q96GC6",
  "term_id": "GO:0000978",
  "gene_symbol": "ZNF274",
  "term_label": "RNA polymerase II cis-regulatory region sequence-specific DNA binding"
}